epigenetic programming in the endosperm [GO:0141044] (biological process) References: PMID:10580004, PMID:16469697, PMID:16527743, PMID:18700816, PMID:28118754 Relationships: is a type of GO:0044725 Definition: The global programming of epigenetic modifications following binucleate central cell fertilization. This involves DNA methylation at the silent allele. In the endosperm, maternal genomes are hypomethylated compared with the paternal genome. Also known as: epigenetic reprogramming in the endosperm